dopamine:sodium symporter activity [GO:0005330] (MF) References: PMID:21752877, PMID:22519513 Sources: TC:2.A.22.1.3 Definition: Enables the transfer of a solute or solutes from one side of a membrane to the other according to the reaction: dopamine(out) + Na+(out) + Cl-(out)= dopamine(in) + Na+(in) + Cl-(in). Also known as: dopamine transmembrane transporter activity, dopamine:sodium:chloride symporter activity, sodium/dopamine symporter activity Relationships: is a type of monoamine transmembrane transporter activity [GO:0008504]; is a type of sodium:chloride symporter activity [GO:0015378]; is part of dopamine uptake [GO:0090494]